{
  "gene_symbol": "KDM4A",
  "gene_name": "Lysine-specific demethylase 4A",
  "term_label": "nucleus",
  "term_id": "GO:0005634",
  "gene": "UniProtKB:O75164"
}